{
  "gene_name": "UDP-glucuronosyltransferase 1A8",
  "gene": "UniProtKB:Q9HAW9",
  "gene_symbol": "UGT1A8",
  "term_label": "cellular response to glucocorticoid stimulus",
  "term_id": "GO:0071385"
}